{
  "gene_symbol": "RUNX2",
  "term_label": "ossification",
  "term_id": "GO:0001503",
  "gene_name": "Runt-related transcription factor 2",
  "gene": "UniProtKB:Q13950"
}